positive regulation of myeloid leukocyte cytokine production involved in immune response [GO:0061081] (biological process) Definition: Any process that modulates the rate, frequency, or extent of the production of a cytokine that contributes to the immune response. Subtypes: positive regulation of myeloid dendritic cell cytokine production [GO:0002735], positive regulation of mast cell cytokine production [GO:0032765], positive regulation of macrophage cytokine production [GO:0060907] Also known as: positive regulation of myeloid cell cytokine production involved in immune response Relationships: is_a positive regulation of cytokine production involved in immune response [GO:0002720]; positively regulates GO:0061082 Sources: GOC:BHF, GOC:dph